{
  "term_id": "GO:0000981",
  "gene_name": "Transcription factor EC",
  "gene": "UniProtKB:O14948",
  "gene_symbol": "TFEC",
  "term_label": "DNA-binding transcription factor activity, RNA polymerase II-specific"
}